{
  "gene_symbol": "HTR2B",
  "term_label": "chemical synaptic transmission",
  "gene": "UniProtKB:P41595",
  "gene_name": "5-hydroxytryptamine receptor 2B",
  "term_id": "GO:0007268"
}